periodic partitioning [GO:0007365] (biological process) Relationships: is a type of regionalization [GO:0003002]; is part of blastoderm segmentation [GO:0007350] Note: Note that examples of periodic partitions are tagmata, segments or parasegments. Sources: GOC:dph, GOC:isa_complete, GOC:ma Subtypes: periodic partitioning by pair rule gene [GO:0007366], segment polarity determination [GO:0007367] Definition: The regionalization process that divides the spatial regions of an embryo into serially repeated regions.